{
  "term_label": "neuron projection development",
  "gene": "UniProtKB:Q92729",
  "gene_name": "Receptor-type tyrosine-protein phosphatase U",
  "gene_symbol": "PTPRU",
  "term_id": "GO:0031175"
}